{
  "gene_name": "Putative coiled-coil domain-containing protein 195",
  "gene_symbol": "CCDC195",
  "gene": "UniProtKB:A0A1B0GUA6",
  "term_id": "UNKNOWN:0003",
  "term_label": "Unknown cellular component"
}